{
  "term_id": "GO:0005737",
  "gene_name": "Protein unc-45 homolog A",
  "gene_symbol": "UNC45A",
  "gene": "UniProtKB:Q9H3U1",
  "term_label": "cytoplasm"
}